regulation of muscle adaptation [GO:0043502] (BP) Relationships: is a type of regulation of response to stimulus [GO:0048583]; is_a regulation of muscle system process [GO:0090257]; regulates GO:0043500 Definition: Any process that modulates the frequency, rate or extent of muscle adaptation. Sources: GOC:go_curators, GOC:mtg_muscle Subtypes: regulation of cardiac muscle hypertrophy [GO:0010611], regulation of cardiac muscle adaptation [GO:0010612], regulation of skeletal muscle adaptation [GO:0014733], GO:0014735, regulation of muscle hyperplasia [GO:0014738], GO:0014744, negative regulation of muscle adaptation [GO:0014745], regulation of smooth muscle hypertrophy [GO:1905147] Also known as: regulation of muscle plasticity